{
  "gene": "UniProtKB:Q8TEW0",
  "gene_symbol": "PARD3",
  "gene_name": "Partitioning defective 3 homolog",
  "term_id": "GO:0035091",
  "term_label": "phosphatidylinositol binding"
}